hydrolase activity, acting on acid carbon-carbon bonds [GO:0016822] (molecular function) Subtypes: GO:0016823, 6-hydroxycyclohex-1-ene-1-carboxyl-CoA hydratase activity [GO:0018807] Sources: GOC:jl Relationships: is_a hydrolase activity [GO:0016787] Definition: Catalysis of the hydrolysis of any acid carbon-carbon bond.